anthocyanidin 3-O-glucoside 6''-O-acyltransferase activity [GO:0102453] (MF) Sources: GOC:pz, RHEA:35411 Relationships: is a type of acyltransferase activity, transferring groups other than amino-acyl groups [GO:0016747] Definition: Catalysis of the reaction: 4-coumaryl-CoA + H+ + an anthocyanidin-3-O-beta-D-glucoside = coenzyme A + H+ + an anthocyanidin-3-O-[6-O-(hydroxycinnamoyl)-beta-D-glucoside].